{
  "gene_name": "Trichoplein keratin filament-binding protein",
  "gene": "UniProtKB:Q9BT92",
  "term_id": "GO:0006915",
  "term_label": "apoptotic process",
  "gene_symbol": "TCHP"
}